{
  "gene_name": "Latent-transforming growth factor beta-binding protein 2",
  "gene_symbol": "LTBP2",
  "term_label": "extracellular matrix",
  "gene": "UniProtKB:Q14767",
  "term_id": "GO:0031012"
}